boss receptor activity [GO:0008288] (molecular function) Also known as: sevenless receptor activity Definition: Combining with a protein bride of sevenless (boss) and transmitting the signal from one side of the membrane to the other to initiate a change in cell activity by catalysis of the reaction: ATP + a protein-L-tyrosine = ADP + a protein-L-tyrosine phosphate. Relationships: is a type of transmembrane receptor protein tyrosine kinase activity [GO:0004714] Sources: GOC:jl, GOC:signaling